{
  "term_label": "Unknown biological process",
  "term_id": "UNKNOWN:0002",
  "gene_name": "Pogo transposable element with KRAB domain",
  "gene": "UniProtKB:Q9P215",
  "gene_symbol": "POGK"
}